{
  "gene": "UniProtKB:Q9NXG0",
  "gene_symbol": "CNTLN",
  "gene_name": "Centlein",
  "term_id": "GO:0005814",
  "term_label": "centriole"
}